{
  "gene_symbol": "CTNNB1",
  "term_label": "alpha-catenin binding",
  "gene": "UniProtKB:P35222",
  "term_id": "GO:0045294",
  "gene_name": "Catenin beta-1"
}